purine deoxyribonucleoside monophosphate biosynthetic process [GO:0009171] (biological process) Also known as: purine deoxyribonucleoside monophosphate anabolism, purine deoxyribonucleoside monophosphate biosynthesis, purine deoxyribonucleoside monophosphate formation, purine deoxyribonucleoside monophosphate synthesis Subtypes: dAMP biosynthetic process [GO:0006170], dGMP biosynthetic process [GO:0006181], dIMP salvage [GO:0106385] Definition: The chemical reactions and pathways resulting in the formation of purine deoxyribonucleoside monophosphate, a compound consisting of a purine base linked to a deoxyribose sugar esterified with phosphate on the sugar. Relationships: is a type of GO:0009127; is a type of deoxyribonucleoside monophosphate biosynthetic process [GO:0009157]; is a type of purine deoxyribonucleoside monophosphate metabolic process [GO:0009170] Sources: GOC:go_curators, ISBN:0198506732